{
  "term_id": "GO:0044209",
  "gene_name": "Adenine phosphoribosyltransferase",
  "term_label": "AMP salvage",
  "gene_symbol": "APRT",
  "gene": "UniProtKB:P07741"
}